{
  "gene_symbol": "SLC13A2",
  "term_label": "plasma membrane",
  "term_id": "GO:0005886",
  "gene_name": "Solute carrier family 13 member 2",
  "gene": "UniProtKB:Q13183"
}